cytokinin riboside 5'-monophosphate phosphoribohydrolase activity [GO:0102682] (molecular function) Also known as: N6-(Delta2-isopentenyl)-adenosine 5'-monophosphate phosphoribohydrolase activity Relationships: is a type of hydrolase activity, hydrolyzing N-glycosyl compounds [GO:0016799] Sources: GOC:pz, RHEA:48560 Definition: Catalysis of the reaction: N(6)-(dimethylallyl)adenosine 5'-phosphate + H2O = N(6)-dimethylallyladenine + D-ribose 5-phosphate.